phosphatidylinositol monophosphate phosphatase activity [GO:0052744] (molecular function) Definition: Catalysis of the reaction: phosphatidyl-1D-myo-inositol monophosphate + H2O = phosphatidylinositol + phosphate. Subtypes: phosphatidylinositol-3-phosphate phosphatase activity [GO:0004438], GO:0043812, phosphatidylinositol-5-phosphate phosphatase activity [GO:0102091] Relationships: is a type of phosphatidylinositol phosphate phosphatase activity [GO:0052866] Sources: GOC:ai